{
  "gene": "UniProtKB:Q8NH79",
  "term_id": "UNKNOWN:0002",
  "gene_name": "Olfactory receptor 6X1",
  "gene_symbol": "OR6X1",
  "term_label": "Unknown biological process"
}